{
  "term_label": "nucleus",
  "term_id": "GO:0005634",
  "gene_name": "Oxidation resistance protein 1",
  "gene": "UniProtKB:Q8N573",
  "gene_symbol": "OXR1"
}